{
  "term_label": "Unknown cellular component",
  "gene": "UniProtKB:Q68CJ6",
  "gene_symbol": "NUGGC",
  "gene_name": "Nuclear GTPase SLIP-GC",
  "term_id": "UNKNOWN:0003"
}